oximinotransferase activity [GO:0050206] (molecular function) Sources: RHEA:11624 Also known as: oximase activity, oximinotransaminase activity, pyruvate-acetone oximinotransferase activity, transoximase activity, transoximinase activity Relationships: is a type of transferase activity, transferring nitrogenous groups [GO:0016769] Definition: Catalysis of the reaction: 2-(hydroxyimino)propanoate + acetone = acetone oxime + pyruvate.